{
  "gene_symbol": "SLC1A4",
  "gene_name": "Neutral amino acid transporter A",
  "term_id": "GO:0015194",
  "term_label": "L-serine transmembrane transporter activity",
  "gene": "UniProtKB:P43007"
}